{
  "gene_name": "Condensin-2 complex subunit D3",
  "gene_symbol": "NCAPD3",
  "gene": "UniProtKB:P42695",
  "term_id": "GO:0010032",
  "term_label": "meiotic chromosome condensation"
}